{
  "term_id": "GO:0000785",
  "gene_symbol": "PPP1R10",
  "gene": "UniProtKB:Q96QC0",
  "gene_name": "Serine_threonine-protein phosphatase 1 regulatory subunit 10",
  "term_label": "chromatin"
}